pantothenate import across plasma membrane [GO:0098717] (biological process) Definition: The directed movement of pantothenate from outside of a cell, across the plasma membrane and into the cytosol. Also known as: pantothenate import into cell, pantothenate import Sources: GOC:dos Relationships: is a type of pantothenate transmembrane transport [GO:0015887]; is a type of import across plasma membrane [GO:0098739]